response to silicon dioxide [GO:0034021] (biological process) Also known as: response to silica, response to silox Subtypes: cellular response to silicon dioxide [GO:0071251] Sources: GOC:sl Definition: Any process that results in a change in state or activity of a cell or an organism (in terms of movement, secretion, enzyme production, gene expression, etc.) as a result of a silicon dioxide stimulus. Relationships: is a type of GO:1901700